amino acid transmembrane transporter activity [GO:0015171] (molecular function) Subtypes: glutamate-gated receptor activity [GO:0004970], amino acid:monoatomic cation symporter activity [GO:0005416], acidic amino acid transmembrane transporter activity [GO:0015172], GO:0015174, GO:0015175, L-amino acid transmembrane transporter activity [GO:0015179], gamma-aminobutyric acid transmembrane transporter activity [GO:0015185], ABC-type amino acid transporter activity [GO:0015424], D-amino acid transmembrane transporter activity [GO:0042943], arginine:ornithine antiporter activity [GO:0043858], GO:0043862, methionine transmembrane transporter activity [GO:0043865], GO:0043872, 5-aminolevulinic acid transmembrane transporter activity [GO:0140485], amino acid:monoatomic cation antiporter activity [GO:0140848] Also known as: amino acid transporter activity, amino acid permease activity, amino acid/choline transmembrane transporter activity, general amino acid permease activity, hydroxy/aromatic amino acid permease activity Relationships: is a type of transmembrane transporter activity [GO:0022857]; is part of GO:0003333 Definition: Enables the transfer of amino acids from one side of a membrane to the other. Amino acids are organic molecules that contain an amino group and a carboxyl group. Sources: GOC:ai, GOC:mtg_transport, ISBN:0815340729